{
  "gene_symbol": "ZSCAN26",
  "term_id": "GO:0000981",
  "gene_name": "Zinc finger and SCAN domain-containing protein 26",
  "gene": "UniProtKB:Q16670",
  "term_label": "DNA-binding transcription factor activity, RNA polymerase II-specific"
}